{
  "term_label": "membrane",
  "term_id": "GO:0016020",
  "gene": "UniProtKB:Q9BXJ8",
  "gene_name": "Ion channel TACAN",
  "gene_symbol": "TMEM120A"
}